prostate gland growth [GO:0060736] (biological process) Relationships: is a type of developmental process involved in reproduction [GO:0003006]; is a type of GO:0035265; is part of prostate gland development [GO:0030850] Definition: The increase in size or mass of the prostate gland where the increase in size or mass has the specific outcome of the progression of the gland, from its formation to its mature state. Sources: GOC:dph Subtypes: GO:0060737